proton motive force-driven ATP synthesis [GO:0015986] (biological process) Definition: The chemical reactions and pathways resulting in the formation of ATP driven by transport of protons across a membrane to generate an electrochemical gradient (proton-motive force). Relationships: is a type of GO:0006754 Sources: GOC:vw Subtypes: proton motive force-driven mitochondrial ATP synthesis [GO:0042776], proton motive force-driven plasma membrane ATP synthesis [GO:0042777] Also known as: chemiosmosis, ATP synthesis coupled proton transport